{
  "gene": "UniProtKB:Q92633",
  "term_id": "GO:0005886",
  "term_label": "plasma membrane",
  "gene_symbol": "LPAR1",
  "gene_name": "Lysophosphatidic acid receptor 1"
}